high-affinity zinc transmembrane transporter activity [GO:0000006] (MF) Definition: Enables the transfer of zinc ions (Zn2+) from one side of a membrane to the other, probably powered by proton motive force. In high-affinity transport the transporter is able to bind the solute even if it is only present at very low concentrations. Relationships: is_a GO:0005385 Also known as: high affinity zinc uptake transmembrane transporter activity, high-affinity zinc uptake transmembrane transporter activity Sources: TC:2.A.5.1.1